{
  "gene": "UniProtKB:P22392",
  "gene_symbol": "NME2",
  "term_id": "GO:0004550",
  "term_label": "nucleoside diphosphate kinase activity",
  "gene_name": "Nucleoside diphosphate kinase B"
}